{
  "term_label": "Unknown molecular function",
  "gene_name": "Probable G-protein coupled receptor 139",
  "term_id": "UNKNOWN:0001",
  "gene": "UniProtKB:Q6DWJ6",
  "gene_symbol": "GPR139"
}